{
  "gene": "UniProtKB:O00311",
  "term_id": "GO:0005634",
  "gene_symbol": "CDC7",
  "term_label": "nucleus",
  "gene_name": "Cell division cycle 7-related protein kinase"
}